{
  "gene": "UniProtKB:A6NFA0",
  "gene_symbol": "SPATA31F3",
  "term_id": "UNKNOWN:0003",
  "gene_name": "Protein SPATA31F3",
  "term_label": "Unknown cellular component"
}